{
  "gene_symbol": "HRH2",
  "term_id": "GO:0007268",
  "gene_name": "Histamine H2 receptor",
  "term_label": "chemical synaptic transmission",
  "gene": "UniProtKB:P25021"
}